{
  "gene": "UniProtKB:Q9UJU2",
  "gene_name": "Lymphoid enhancer-binding factor 1",
  "gene_symbol": "LEF1",
  "term_label": "DNA-binding transcription factor activity, RNA polymerase II-specific",
  "term_id": "GO:0000981"
}